6-oxocineole dehydrogenase activity [GO:0047597] (molecular function) Relationships: is a type of oxidoreductase activity, acting on paired donors, with incorporation or reduction of molecular oxygen, NAD(P)H as one donor, and incorporation of one atom of oxygen [GO:0016709] Sources: EC:1.14.13.51, RHEA:24324 Also known as: 6-oxocineole oxygenase activity, 6-oxocineole,NADPH:oxygen oxidoreductase activity Definition: Catalysis of the reaction: 6-oxocineole + H+ + NADPH + O2 = 1,6,6-trimethyl-2,7-dioxabicyclo[3.2.2]nonan-3-one + H2O + NADP+.